{
  "term_label": "GTPase activator activity",
  "gene_name": "Ras GTPase-activating-like protein IQGAP1",
  "gene": "UniProtKB:P46940",
  "term_id": "GO:0005096",
  "gene_symbol": "IQGAP1"
}